{
  "term_id": "GO:0005615",
  "gene_name": "Phospholipase A2 group XV",
  "term_label": "extracellular space",
  "gene": "UniProtKB:Q8NCC3",
  "gene_symbol": "PLA2G15"
}